{
  "gene": "UniProtKB:Q5T036",
  "gene_name": "Uncharacterized protein FAM120AOS",
  "gene_symbol": "FAM120AOS",
  "term_label": "Unknown molecular function",
  "term_id": "UNKNOWN:0001"
}